inner ear development [GO:0048839] (BP) Definition: The process whose specific outcome is the progression of the inner ear over time, from its formation to the mature structure. Relationships: is a type of anatomical structure development [GO:0048856]; BFO_0000050 ear development [GO:0043583] Subtypes: otic vesicle development [GO:0071599] Sources: GOC:sr